{
  "term_label": "Golgi membrane",
  "gene_name": "Formimidoyltransferase-cyclodeaminase",
  "gene": "UniProtKB:O95954",
  "term_id": "GO:0000139",
  "gene_symbol": "FTCD"
}